{
  "term_id": "GO:0005739",
  "term_label": "mitochondrion",
  "gene_symbol": "MTRES1",
  "gene_name": "Mitochondrial transcription rescue factor 1",
  "gene": "UniProtKB:Q9P0P8"
}